{
  "term_id": "GO:0030552",
  "term_label": "cAMP binding",
  "gene_name": "cAMP-dependent protein kinase type II-beta regulatory subunit",
  "gene": "UniProtKB:P31323",
  "gene_symbol": "PRKAR2B"
}